condensin complex [GO:0000796] (cellular component) Also known as: 13S condensin complex, 8S condensin complex, Smc2-Smc4 complex, condensin I complex, condensin core heterodimer, nuclear condensin complex, SMC complex Relationships: is a type of protein-containing complex [GO:0032991]; is part of GO:0005694 Definition: A multisubunit protein complex that plays a central role in chromosome condensation in meiosis and mitosis. References: PMID:17268547, PMID:21795393 Sources: GOC:elh